paraxial mesoderm formation [GO:0048341] (BP) Definition: The process that gives rise to the paraxial mesoderm. This process pertains to the initial formation of the structure from unspecified parts. Sources: GOC:dgh Relationships: is a type of mesoderm formation [GO:0001707]; is part of paraxial mesoderm morphogenesis [GO:0048340]